{
  "term_id": "GO:0004016",
  "term_label": "adenylate cyclase activity",
  "gene": "UniProtKB:O43306",
  "gene_symbol": "ADCY6",
  "gene_name": "Adenylate cyclase type 6"
}